{
  "gene": "UniProtKB:Q02575",
  "gene_name": "Helix-loop-helix protein 1",
  "gene_symbol": "NHLH1",
  "term_label": "DNA-binding transcription factor activity, RNA polymerase II-specific",
  "term_id": "GO:0000981"
}